{
  "gene_name": "Rho guanine nucleotide exchange factor 1",
  "term_id": "GO:0007186",
  "term_label": "G protein-coupled receptor signaling pathway",
  "gene": "UniProtKB:Q92888",
  "gene_symbol": "ARHGEF1"
}